{
  "term_id": "GO:0140566",
  "gene_name": "E3 ubiquitin-protein ligase Jade-2",
  "gene_symbol": "JADE2",
  "term_label": "histone reader activity",
  "gene": "UniProtKB:Q9NQC1"
}